{
  "gene_symbol": "CALML5",
  "term_id": "GO:0005737",
  "gene": "UniProtKB:Q9NZT1",
  "gene_name": "Calmodulin-like protein 5",
  "term_label": "cytoplasm"
}